1,3-propanediol dehydrogenase activity [GO:0047516] (molecular function) Relationships: is a type of oxidoreductase activity, acting on the CH-OH group of donors, NAD or NADP as acceptor [GO:0016616] Also known as: 1,3-PD:NAD+ oxidoreductase activity, 1,3-propanediol oxidoreductase activity, 1,3-propanediol:NAD+ oxidoreductase activity, 3-hydroxypropionaldehyde reductase activity, propane-1,3-diol:NAD+ 1-oxidoreductase activity Sources: EC:1.1.1.202, MetaCyc:13-PROPANEDIOL-DEHYDROGENASE-RXN Definition: Catalysis of the reaction: propane-1,3-diol + NAD+ = 3-hydroxypropanal + NADH + H+.